{
  "gene_symbol": "IL36G",
  "gene_name": "Interleukin-36 gamma",
  "term_label": "inflammatory response",
  "term_id": "GO:0006954",
  "gene": "UniProtKB:Q9NZH8"
}